{
  "gene_symbol": "CDH4",
  "gene_name": "Cadherin-4",
  "term_label": "adherens junction organization",
  "term_id": "GO:0034332",
  "gene": "UniProtKB:P55283"
}